{
  "term_label": "Unknown molecular function",
  "term_id": "UNKNOWN:0001",
  "gene": "UniProtKB:Q96PG2",
  "gene_name": "Membrane-spanning 4-domains subfamily A member 10",
  "gene_symbol": "MS4A10"
}